{
  "term_label": "fatty acid biosynthetic process",
  "gene_symbol": "PNLIP",
  "gene_name": "Pancreatic triacylglycerol lipase",
  "gene": "UniProtKB:P16233",
  "term_id": "GO:0006633"
}